{
  "gene_symbol": "Q6ZN92",
  "gene": "UniProtKB:Q6ZN92",
  "term_label": "dUMP biosynthetic process",
  "term_id": "GO:0006226",
  "gene_name": "Putative inactive deoxyuridine 5'-triphosphate nucleotidohydrolase-like protein FLJ16323"
}